intracellular pH reduction [GO:0051452] (biological process) Sources: GOC:ai Regulation: regulated by regulation of cellular pH reduction [GO:0032847]; negatively regulated by negative regulation of cellular pH reduction [GO:0032848]; positively regulated by positive regulation of cellular pH reduction [GO:0032849] Also known as: cell pH reduction, cellular acidification, reduction of cellular pH, reduction of pH in cell, intracellular acidification Subtypes: vacuolar acidification [GO:0007035], positive regulation of cellular pH reduction [GO:0032849], GO:0048388, GO:0061795, GO:0090383 Definition: Any process that reduces the internal pH of a cell, measured by the concentration of the hydrogen ion. Relationships: is a type of regulation of intracellular pH [GO:0051453]